methylation-dependent protein binding [GO:0140034] (molecular function) Relationships: is a type of modification-dependent protein binding [GO:0140030] References: PMID:26060076 Note: This term should only be used when the binding is shown to require methylation of the target protein: the interaction needs to be tested with and without the PTM. The binding does not need to be at the site of methylation. It may be that the methylation causes a conformational change that allows binding of the protein to another region; this type of methylation-dependent protein binding is valid for annotation to this term. Definition: Binding to a protein upon methylation of the target protein.